lactaldehyde reductase activity [GO:0008912] (MF) Also known as: propanediol oxidoreductase activity, (R)- or (S)-propane-1,2-diol:NAD+ oxidoreductase activity, lactaldehyde:propanediol oxidoreductase activity, propanediol:nicotinamide adenine dinucleotide (NAD) oxidoreductase activity Subtypes: R-lactaldehyde reductase activity [GO:0052660], S-lactaldehyde reductase activity [GO:0052661] Sources: EC:1.1.1.77 Relationships: is a type of oxidoreductase activity, acting on the CH-OH group of donors, NAD or NADP as acceptor [GO:0016616] Definition: Catalysis of the reaction: propane-1,2-diol + NAD+ = lactaldehyde + NADH + H+.